regulation of mitotic cell cycle, embryonic [GO:0009794] (biological process) Sources: GOC:dph, GOC:go_curators, GOC:tb Subtypes: regulation of preblastoderm mitotic cell cycle [GO:0007347], regulation of syncytial blastoderm mitotic cell cycle [GO:0007348], negative regulation of mitotic cell cycle, embryonic [GO:0045976], GO:0045977 Also known as: embryonic mitotic cell cycle modulation, embryonic mitotic cell cycle regulation, modulation of embryonic mitotic cell cycle progression, regulation of embryonic mitotic cell cycle, regulation of embryonic mitotic cell cycle progression, regulation of progression through embryonic mitotic cell cycle, embryonic mitotic cell cycle regulator Relationships: is a type of regulation of mitotic cell cycle [GO:0007346]; regulates mitotic cell cycle, embryonic [GO:0045448] Definition: Any process that modulates the frequency, rate or extent of replication and segregation of genetic material in the embryo.